creatinine deaminase activity [GO:0047790] (molecular function) Sources: EC:3.5.4.21, MetaCyc:CREATININE-DEAMINASE-RXN Definition: Catalysis of the reaction: creatinine + H2O = N-methylhydantoin + NH3. Also known as: creatinine hydrolase, creatinine desiminase activity, creatinine iminohydrolase activity Relationships: is a type of hydrolase activity, acting on carbon-nitrogen (but not peptide) bonds, in cyclic amidines [GO:0016814]; is a type of deaminase activity [GO:0019239]